{
  "gene": "UniProtKB:Q9BRH9",
  "gene_name": "Zinc finger protein 251",
  "term_id": "GO:0000981",
  "term_label": "DNA-binding transcription factor activity, RNA polymerase II-specific",
  "gene_symbol": "ZNF251"
}